regulation of amino acid transmembrane transport [GO:1903789] (biological process) Definition: Any process that modulates the frequency, rate or extent of amino acid transmembrane transport. References: PMID:16115814 Sources: GOC:TermGenie, GO_REF:0000058 Also known as: regulation of amino acid membrane transport Relationships: is a type of regulation of transmembrane transport [GO:0034762]; is a type of regulation of amino acid transport [GO:0051955]; regulates amino acid transmembrane transport [GO:0003333] Subtypes: regulation of amino acid import across plasma membrane [GO:0010958], GO:0080143